pronuclear migration [GO:0035046] (biological process) Definition: The directed movement of the male and female pronuclei towards each other prior to their fusion. References: PMID:9199363 Sources: GOC:bf Relationships: is a type of nuclear migration [GO:0007097]; is part of single fertilization [GO:0007338]